{
  "gene_name": "Tubulin gamma-2 chain",
  "term_id": "GO:0005819",
  "gene_symbol": "TUBG2",
  "gene": "UniProtKB:Q9NRH3",
  "term_label": "spindle"
}